{
  "term_label": "RNA polymerase II cis-regulatory region sequence-specific DNA binding",
  "gene": "UniProtKB:P48431",
  "term_id": "GO:0000978",
  "gene_name": "Transcription factor SOX-2",
  "gene_symbol": "SOX2"
}